{
  "term_id": "GO:0003712",
  "gene": "UniProtKB:Q92925",
  "term_label": "transcription coregulator activity",
  "gene_name": "SWI_SNF-related matrix-associated actin-dependent regulator of chromatin subfamily D member 2",
  "gene_symbol": "SMARCD2"
}